{
  "gene_symbol": "RFTN1",
  "gene": "UniProtKB:Q14699",
  "term_label": "Unknown cellular component",
  "term_id": "UNKNOWN:0003",
  "gene_name": "Raftlin"
}